{
  "term_id": "GO:0051959",
  "gene_symbol": "HOOK3",
  "term_label": "dynein light intermediate chain binding",
  "gene": "UniProtKB:Q86VS8",
  "gene_name": "Protein Hook homolog 3"
}